{
  "term_label": "protein-macromolecule adaptor activity",
  "gene_name": "Epidermal growth factor receptor substrate 15-like 1",
  "term_id": "GO:0030674",
  "gene_symbol": "EPS15L1",
  "gene": "UniProtKB:Q9UBC2"
}